{
  "term_id": "GO:0030527",
  "gene": "UniProtKB:Q93077",
  "gene_symbol": "H2AC6",
  "term_label": "structural constituent of chromatin",
  "gene_name": "Histone H2A type 1-C"
}